{
  "gene_name": "Kinesin-like protein KIF18B",
  "gene_symbol": "KIF18B",
  "term_id": "GO:0008017",
  "term_label": "microtubule binding",
  "gene": "UniProtKB:Q86Y91"
}